xanthine binding [GO:0160050] (molecular function) Definition: Binding to xanthine, a purine base. Relationships: is a type of GO:0002060 References: PMID:32345632, PMID:34125892